{
  "term_label": "endosome membrane",
  "gene_symbol": "RAB15",
  "gene": "UniProtKB:P59190",
  "term_id": "GO:0010008",
  "gene_name": "Ras-related protein Rab-15"
}